{
  "term_label": "Unknown cellular component",
  "term_id": "UNKNOWN:0003",
  "gene_name": "Myelin transcription factor 1",
  "gene": "UniProtKB:Q01538",
  "gene_symbol": "MYT1"
}